{
  "gene": "UniProtKB:Q8NC06",
  "gene_name": "Acyl-CoA-binding domain-containing protein 4",
  "term_label": "fatty acid metabolic process",
  "term_id": "GO:0006631",
  "gene_symbol": "ACBD4"
}